2-amino-4-hydroxy-6-hydroxymethyldihydropteridine diphosphokinase activity [GO:0003848] (molecular function) Definition: Catalysis of the reaction: 2-amino-4-hydroxy-6-hydroxymethyl-7,8-dihydropteridine + ATP = (2-amino-4-hydroxy-7,8-dihydropteridin-6-yl)methyl diphosphate + AMP + 2 H+. Sources: EC:2.7.6.3, RHEA:11412 Also known as: 2-amino-4-hydroxy-6-hydroxymethyldihydropteridine pyrophosphokinase activity, 6-hydroxymethyl-7,8-dihydropterin diphosphokinase activity, 6-hydroxymethyl-7,8-dihydropterin pyrophosphokinase activity, 7,8-dihydro-6-hydroxymethylpterin diphosphokinase activity, 7,8-dihydro-6-hydroxymethylpterin pyrophosphokinase activity, 7,8-dihydroxymethylpterin-pyrophosphokinase activity, ATP:2-amino-4-hydroxy-6-hydroxymethyl-7,8-dihydropteridine 6'-diphosphotransferase activity, H2-pteridine-CH2OH pyrophosphokinase activity, HPPK, hydroxymethyldihydropteridine pyrophosphokinase activity Relationships: is a type of diphosphotransferase activity [GO:0016778]